negative regulation of [2Fe-2S] cluster assembly [GO:1900488] (biological process) Relationships: is a type of regulation of [2Fe-2S] cluster assembly [GO:1900487]; is a type of negative regulation of iron-sulfur cluster assembly [GO:1903330]; negatively regulates [2Fe-2S] cluster assembly [GO:0044571] Definition: Any process that stops, prevents or reduces the frequency, rate or extent of [2Fe-2S] cluster assembly. Also known as: down regulation of 2Fe-2S cluster assembly, down regulation of [2Fe-2S] cluster assembly, down-regulation of 2Fe-2S cluster assembly, down-regulation of [2Fe-2S] cluster assembly, downregulation of 2Fe-2S cluster assembly, downregulation of [2Fe-2S] cluster assembly, negative regulation of 2Fe-2S cluster assembly, inhibition of 2Fe-2S cluster assembly, inhibition of [2Fe-2S] cluster assembly, down regulation of [2Fe-2S] cluster biosynthetic process, down-regulation of [2Fe-2S] cluster biosynthetic process, downregulation of [2Fe-2S] cluster biosynthetic process, inhibition of [2Fe-2S] cluster biosynthetic process, negative regulation of [2Fe-2S] cluster biosynthetic process Sources: GOC:TermGenie, GOC:mengo_curators